{
  "gene_symbol": "ITGB1",
  "term_id": "GO:0033627",
  "gene": "UniProtKB:P05556",
  "term_label": "cell adhesion mediated by integrin",
  "gene_name": "Integrin beta-1"
}